{
  "gene_symbol": "RBM14",
  "term_label": "nuclear speck",
  "gene": "UniProtKB:Q96PK6",
  "gene_name": "RNA-binding protein 14",
  "term_id": "GO:0016607"
}